{
  "term_label": "aldose reductase (NADPH) activity",
  "term_id": "GO:0004032",
  "gene_name": "Aldo-keto reductase family 1 member B15",
  "gene_symbol": "AKR1B15",
  "gene": "UniProtKB:C9JRZ8"
}